{
  "gene_symbol": "ZNF722",
  "gene_name": "Zinc finger protein 722",
  "term_id": "GO:0006355",
  "term_label": "regulation of DNA-templated transcription",
  "gene": "UniProtKB:A0A1W2PQL4"
}